C5a anaphylatoxin chemotactic receptor binding [GO:0031714] (molecular function) Relationships: is a type of G protein-coupled receptor binding [GO:0001664] Sources: GOC:mah, GOC:nln Subtypes: GO:0031715 Definition: Binding to a C5a anaphylatoxin chemotactic receptor. Also known as: C5a anaphylatoxin chemotactic receptor ligand